{
  "gene_symbol": "ASAP2",
  "term_label": "GTPase activator activity",
  "term_id": "GO:0005096",
  "gene_name": "Arf-GAP with SH3 domain, ANK repeat and PH domain-containing protein 2",
  "gene": "UniProtKB:O43150"
}